{
  "gene_name": "GRB2-related adapter protein",
  "gene": "UniProtKB:Q13588",
  "term_id": "GO:0005654",
  "gene_symbol": "GRAP",
  "term_label": "nucleoplasm"
}